{
  "gene_name": "Leucine-rich repeat-containing protein 7",
  "gene_symbol": "LRRC7",
  "term_id": "GO:0043194",
  "gene": "UniProtKB:Q96NW7",
  "term_label": "axon initial segment"
}